{
  "term_label": "olfactory receptor activity",
  "term_id": "GO:0004984",
  "gene_name": "Olfactory receptor 5H6",
  "gene_symbol": "OR5H6",
  "gene": "UniProtKB:Q8NGV6"
}